alphaX-beta2 integrin-ICAM-4 complex [GO:0071132] (cellular component) Also known as: ITGAX-ITGB2-ICAM4 complex Definition: A protein complex that consists of an alphaX-beta2 integrin complex bound to intercellular adhesion molecule 4. Relationships: is a type of plasma membrane protein complex [GO:0098797] References: PMID:16985175